methanesulfonic acid metabolic process [GO:0018926] (BP) Also known as: methanesulfonic acid metabolism, methanesulphonic acid metabolic process, methanesulphonic acid metabolism Relationships: is a type of xenobiotic metabolic process [GO:0006805]; is a type of GO:0019694 Definition: The chemical reactions and pathways involving methanesulfonic acid, a strong acid produced by the oxidation of dimethyl sulfide. Sources: UM-BBD_pathwayID:msa